{
  "gene": "UniProtKB:P35236",
  "term_label": "Unknown cellular component",
  "term_id": "UNKNOWN:0003",
  "gene_symbol": "PTPN7",
  "gene_name": "Tyrosine-protein phosphatase non-receptor type 7"
}